{
  "gene_name": "Putative olfactory receptor 3A4",
  "gene": "UniProtKB:P47883",
  "term_label": "olfactory receptor activity",
  "term_id": "GO:0004984",
  "gene_symbol": "OR3A4P"
}